{
  "gene_symbol": "MCEMP1",
  "term_id": "UNKNOWN:0003",
  "gene": "UniProtKB:Q8IX19",
  "gene_name": "Mast cell-expressed membrane protein 1",
  "term_label": "Unknown cellular component"
}